{
  "term_label": "nucleus",
  "term_id": "GO:0005634",
  "gene_symbol": "NSD3",
  "gene_name": "Histone-lysine N-methyltransferase NSD3",
  "gene": "UniProtKB:Q9BZ95"
}